{
  "gene": "UniProtKB:Q8N9X5",
  "term_label": "Unknown molecular function",
  "term_id": "UNKNOWN:0001",
  "gene_symbol": "LINC02912",
  "gene_name": "Putative protein encoded by LINC02912"
}